{
  "gene": "UniProtKB:Q8N1C3",
  "term_id": "GO:0008503",
  "term_label": "benzodiazepine receptor activity",
  "gene_name": "Gamma-aminobutyric acid receptor subunit gamma-1",
  "gene_symbol": "GABRG1"
}